{
  "term_label": "extracellular space",
  "gene": "UniProtKB:P09382",
  "gene_name": "Galectin-1",
  "term_id": "GO:0005615",
  "gene_symbol": "LGALS1"
}